{
  "gene_symbol": "TMEM219",
  "term_label": "Unknown cellular component",
  "term_id": "UNKNOWN:0003",
  "gene": "UniProtKB:Q86XT9",
  "gene_name": "Insulin-like growth factor-binding protein 3 receptor"
}